{
  "term_label": "transmembrane transporter binding",
  "gene_name": "Leucine-rich repeat-containing protein 55",
  "term_id": "GO:0044325",
  "gene_symbol": "LRRC55",
  "gene": "UniProtKB:Q6ZSA7"
}